{
  "gene_name": "Thyroid hormone receptor beta",
  "gene": "UniProtKB:P10828",
  "term_id": "GO:0002154",
  "gene_symbol": "THRB",
  "term_label": "thyroid hormone receptor signaling pathway"
}